{
  "term_label": "cytosolic small ribosomal subunit",
  "gene_name": "Small ribosomal subunit protein eS21",
  "gene": "UniProtKB:P63220",
  "gene_symbol": "RPS21",
  "term_id": "GO:0022627"
}